{
  "gene": "UniProtKB:P31151",
  "gene_name": "Protein S100-A7",
  "term_label": "endothelial cell migration",
  "term_id": "GO:0043542",
  "gene_symbol": "S100A7"
}